{
  "term_id": "GO:1990756",
  "gene_symbol": "KLHL17",
  "gene": "UniProtKB:Q6TDP4",
  "term_label": "ubiquitin-like ligase-substrate adaptor activity",
  "gene_name": "Kelch-like protein 17"
}